{
  "term_label": "phosphatidylinositol binding",
  "gene": "UniProtKB:Q9BZ72",
  "gene_symbol": "PITPNM2",
  "gene_name": "Membrane-associated phosphatidylinositol transfer protein 2",
  "term_id": "GO:0035091"
}